{
  "term_id": "GO:0010564",
  "gene_symbol": "ANKK1",
  "gene_name": "Ankyrin repeat and protein kinase domain-containing protein 1",
  "term_label": "regulation of cell cycle process",
  "gene": "UniProtKB:Q8NFD2"
}